{
  "term_id": "GO:0006261",
  "gene": "UniProtKB:P35249",
  "term_label": "DNA-templated DNA replication",
  "gene_name": "Replication factor C subunit 4",
  "gene_symbol": "RFC4"
}